{
  "gene_name": "Protein FAM216A",
  "gene": "UniProtKB:Q8WUB2",
  "term_label": "Unknown cellular component",
  "term_id": "UNKNOWN:0003",
  "gene_symbol": "FAM216A"
}